{
  "gene_symbol": "CARS2",
  "term_id": "GO:0004817",
  "gene_name": "Probable cysteine--tRNA ligase, mitochondrial",
  "gene": "UniProtKB:Q9HA77",
  "term_label": "cysteine-tRNA ligase activity"
}